{
  "gene": "UniProtKB:Q99471",
  "term_id": "GO:0016272",
  "gene_name": "Prefoldin subunit 5",
  "term_label": "prefoldin complex",
  "gene_symbol": "PFDN5"
}